{
  "term_id": "UNKNOWN:0002",
  "gene_name": "Serine_threonine-protein kinase ULK4",
  "gene_symbol": "ULK4",
  "gene": "UniProtKB:Q96C45",
  "term_label": "Unknown biological process"
}